{
  "gene": "UniProtKB:Q9UBH6",
  "gene_name": "Solute carrier family 53 member 1",
  "term_label": "cellular response to phosphate starvation",
  "term_id": "GO:0016036",
  "gene_symbol": "XPR1"
}